negative regulation of stomach fundus smooth muscle contraction [GO:0120070] (biological process) References: PMID:15890336 Sources: GOC:sl Relationships: is a type of regulation of stomach fundus smooth muscle contraction [GO:0120068]; is_a negative regulation of gastro-intestinal system smooth muscle contraction [GO:1904305]; negatively regulates stomach fundus smooth muscle contraction [GO:0014825] Definition: Any process that decreases the frequency, rate or extent of any stomach fundus smooth muscle contraction.